{
  "gene": "UniProtKB:Q9Y6B2",
  "gene_name": "EP300-interacting inhibitor of differentiation 1",
  "gene_symbol": "EID1",
  "term_id": "GO:0045892",
  "term_label": "negative regulation of DNA-templated transcription"
}